{
  "gene_symbol": "C11orf68",
  "term_label": "Unknown cellular component",
  "gene_name": "UPF0696 protein C11orf68",
  "term_id": "UNKNOWN:0003",
  "gene": "UniProtKB:Q9H3H3"
}